ethanol biosynthetic process [GO:0006115] (biological process) Also known as: ethanol anabolism, ethanol biosynthesis, ethanol formation, ethanol synthesis Relationships: is_a ethanol metabolic process [GO:0006067]; is a type of primary alcohol biosynthetic process [GO:0034309] Definition: The chemical reactions and pathways resulting in the formation of ethanol, CH3-CH2-OH, a colorless, water-miscible, flammable liquid produced by alcoholic fermentation. Sources: GOC:ai, ISBN:0198506732